{
  "term_id": "GO:0071385",
  "gene_name": "UDP-glucuronosyltransferase 1A3",
  "gene": "UniProtKB:P35503",
  "term_label": "cellular response to glucocorticoid stimulus",
  "gene_symbol": "UGT1A3"
}